negative regulation of granzyme B production [GO:0071662] (biological process) Sources: GOC:mah Relationships: is a type of negative regulation of production of molecular mediator of immune response [GO:0002701]; is a type of regulation of granzyme B production [GO:0071661]; RO_0002212 GO:0071613 Definition: Any process that stops, prevents, or reduces the frequency, rate, or extent of production of granzyme B.